glucose catabolic process to D-lactate and ethanol [GO:0019656] (biological process) Also known as: glucose fermentation to D-lactate and ethanol, heterofermentation, heterofermentative lactate fermentation, heterofermentative pathway, heterolactate fermentation, heterolactic fermentation Relationships: is a type of ethanol metabolic process [GO:0006067]; is a type of glucose catabolic process to lactate [GO:0019659]; is a type of GO:0019662 Sources: GOC:jl, MetaCyc:P122-PWY Definition: The anaerobic chemical reactions and pathways resulting in the enzymatic breakdown of D-glucose to D-lactate and ethanol, yielding energy in the form of adenosine triphosphate (ATP) at the rate of one ATP per glucose molecule.